ribonuclease P complex [GO:0030677] (cellular component) Definition: A ribonucleoprotein complex that catalyzes cleavage of the leader sequence of precursor tRNAs (pre-tRNAs), generating the mature 5' end of tRNAs. Subtypes: GO:0030678, dimeric ribonuclease P complex [GO:0030680], multimeric ribonuclease P complex [GO:0030681] Relationships: is a type of endoribonuclease complex [GO:1902555]; is a type of GO:1990904 Note: Note that chloroplasts possess a complex that is called 'RNase P' because it catalyzes pre-tRNA cleavage, but the chloroplast complex appears not to contain RNA. References: PMID:12045094 Sources: GOC:mah Also known as: RNase P complex